{
  "gene": "UniProtKB:Q9Y5C1",
  "term_label": "triglyceride homeostasis",
  "gene_symbol": "ANGPTL3",
  "gene_name": "Angiopoietin-related protein 3",
  "term_id": "GO:0070328"
}